{
  "gene_name": "Keratin, type II cytoskeletal 75",
  "gene": "UniProtKB:O95678",
  "term_id": "GO:0045109",
  "gene_symbol": "KRT75",
  "term_label": "intermediate filament organization"
}